positive regulation of neurotrophin TRK receptor signaling pathway [GO:0051388] (biological process) Sources: GOC:ai Also known as: positive regulation of NGF receptor signaling pathway, positive regulation of NGF receptor signalling pathway, positive regulation of nerve growth factor receptor signalling pathway, up regulation of nerve growth factor receptor signaling pathway, up-regulation of nerve growth factor receptor signaling pathway, upregulation of nerve growth factor receptor signaling pathway, activation of nerve growth factor receptor signaling pathway, stimulation of nerve growth factor receptor signaling pathway, positive regulation of nerve growth factor receptor signaling pathway Definition: Any process that activates or increases the frequency, rate or extent of the neurotrophin TRK receptor signaling pathway. Relationships: is a type of GO:0009967; is_a regulation of neurotrophin TRK receptor signaling pathway [GO:0051386]; positively regulates neurotrophin TRK receptor signaling pathway [GO:0048011]